ubiquitin-protein transferase activity [GO:0004842] (molecular function) References: PMID:9635407 Sources: GOC:BioGRID, GOC:jh2 Subtypes: ubiquitin protein ligase activity [GO:0061630], ubiquitin conjugating enzyme activity [GO:0061631] Also known as: E2, E3, ubiquitin conjugating enzyme activity, ubiquitin ligase activity, ubiquitin protein ligase activity, ubiquitin protein-ligase activity, ubiquitin-conjugating enzyme activity Relationships: is a type of GO:0019787 Regulation: regulated by regulation of ubiquitin-protein transferase activity [GO:0051438]; positively regulated by positive regulation of ubiquitin-protein transferase activity [GO:0051443]; negatively regulated by negative regulation of ubiquitin-protein transferase activity [GO:0051444]; negatively regulated by ubiquitin-protein transferase inhibitor activity [GO:0055105]; regulated by ubiquitin-protein transferase regulator activity [GO:0055106]; positively regulated by ubiquitin-protein transferase activator activity [GO:0097027] Definition: Catalysis of the transfer of ubiquitin from one protein to another via the reaction X-Ub + Y = Y-Ub + X, where both X-Ub and Y-Ub are covalent linkages.